{
  "term_label": "cytochrome-c oxidase activity",
  "term_id": "GO:0004129",
  "gene_name": "Cytochrome c oxidase subunit 1",
  "gene_symbol": "MT-CO1",
  "gene": "UniProtKB:P00395"
}